sex determination [GO:0007530] (biological process) Relationships: is a type of GO:0003006 Sources: ISBN:0198506732 Subtypes: GO:0007531, primary sex determination [GO:0007538], processes downstream of sex determination signal [GO:0007545], germ-line sex determination [GO:0018992], GO:0018993, female sex determination [GO:0030237], male sex determination [GO:0030238] Definition: Any process that establishes and transmits the specification of sexual status of an individual organism.